{
  "gene_name": "Gamma-crystallin C",
  "term_label": "visual perception",
  "term_id": "GO:0007601",
  "gene": "UniProtKB:P07315",
  "gene_symbol": "CRYGC"
}